{
  "gene_symbol": "HSD3B7",
  "gene": "UniProtKB:Q9H2F3",
  "gene_name": "3 beta-hydroxysteroid dehydrogenase type 7",
  "term_label": "Unknown cellular component",
  "term_id": "UNKNOWN:0003"
}